box H/ACA sno(s)RNA processing [GO:0034964] (biological process) Sources: GOC:krc, GOC:mah Subtypes: box H/ACA sno(s)RNA 3'-end processing [GO:0000495], intronic box H/ACA snoRNA processing [GO:0034966] Relationships: is a type of box H/ACA sno(s)RNA metabolic process [GO:0033979]; is a type of sno(s)RNA processing [GO:0043144] Also known as: box H/ACA sRNA processing, box H/ACA snoRNA processing Definition: Any process involved in the conversion of a primary box H/ACA type small RNA transcript into a mature box H/ACA RNA.